{
  "gene_name": "Fibroblast growth factor 21",
  "term_label": "growth factor activity",
  "gene": "UniProtKB:Q9NSA1",
  "gene_symbol": "FGF21",
  "term_id": "GO:0008083"
}